{
  "gene_symbol": "GALNT18",
  "gene": "UniProtKB:Q6P9A2",
  "term_label": "Golgi apparatus",
  "gene_name": "Polypeptide N-acetylgalactosaminyltransferase 18",
  "term_id": "GO:0005794"
}